{
  "gene_symbol": "ACSL6",
  "gene_name": "Long-chain-fatty-acid--CoA ligase 6",
  "term_label": "very long-chain fatty acid metabolic process",
  "gene": "UniProtKB:Q9UKU0",
  "term_id": "GO:0000038"
}